{
  "gene": "UniProtKB:A6NJJ6",
  "gene_symbol": "C19orf67",
  "term_id": "GO:0001701",
  "term_label": "in utero embryonic development",
  "gene_name": "UPF0575 protein C19orf67"
}